regulation of border follicle cell migration [GO:1903684] (BP) Definition: Any process that modulates the frequency, rate or extent of border follicle cell migration. Subtypes: negative regulation of border follicle cell migration [GO:1903687], positive regulation of border follicle cell migration [GO:1903688] Relationships: is a type of regulation of epithelial cell migration [GO:0010632]; regulates border follicle cell migration [GO:0007298] References: PMID:18394891 Sources: GOC:TermGenie, GOC:als, GO_REF:0000058 Also known as: regulation of border cell migration